{
  "gene": "UniProtKB:P61266",
  "gene_name": "Syntaxin-1B",
  "term_label": "synaptic vesicle fusion to presynaptic active zone membrane",
  "term_id": "GO:0031629",
  "gene_symbol": "STX1B"
}